{
  "gene": "UniProtKB:Q9UGM3",
  "gene_symbol": "DMBT1",
  "term_id": "GO:0050829",
  "gene_name": "Deleted in malignant brain tumors 1 protein",
  "term_label": "defense response to Gram-negative bacterium"
}